{
  "term_id": "UNKNOWN:0001",
  "term_label": "Unknown molecular function",
  "gene": "UniProtKB:P01699",
  "gene_symbol": "IGLV1-44",
  "gene_name": "Immunoglobulin lambda variable 1-44"
}